{
  "gene_symbol": "CCDC69",
  "term_label": "microtubule binding",
  "gene_name": "Coiled-coil domain-containing protein 69",
  "term_id": "GO:0008017",
  "gene": "UniProtKB:A6NI79"
}